{
  "gene_name": "Interferon-induced transmembrane protein 2",
  "term_label": "response to type II interferon",
  "term_id": "GO:0034341",
  "gene": "UniProtKB:Q01629",
  "gene_symbol": "IFITM2"
}